{
  "gene_name": "Thioredoxin, mitochondrial",
  "gene": "UniProtKB:Q99757",
  "term_id": "UNKNOWN:0001",
  "term_label": "Unknown molecular function",
  "gene_symbol": "TXN2"
}